retina vasculature morphogenesis in camera-type eye [GO:0061299] (biological process) Also known as: retinal vasculature morphogenesis Sources: GOC:BHF, GOC:dph Definition: The process in which the vasculature of the retina is generated and organized. Relationships: is a type of anatomical structure morphogenesis [GO:0009653]; is part of GO:0061298 Subtypes: retinal blood vessel morphogenesis [GO:0061304]